{
  "gene_symbol": "NRIP1",
  "term_label": "negative regulation of transcription by RNA polymerase II",
  "term_id": "GO:0000122",
  "gene_name": "Nuclear receptor-interacting protein 1",
  "gene": "UniProtKB:P48552"
}